negative regulation of somatostatin secretion [GO:0090275] (biological process) Definition: Any process that decreases the rate, frequency, extent of the regulated release of somatostatin from secretory granules in the D cells of the pancreas. Sources: GOC:BHF Relationships: is a type of regulation of somatostatin secretion [GO:0090273]; is a type of negative regulation of peptide hormone secretion [GO:0090278]; negatively regulates somatostatin secretion [GO:0070253]